VEGF-activated neuropilin signaling pathway [GO:0038190] (biological process) Also known as: VEGF-Npn-1 signaling, vascular endothelial growth factor-activated neuropilin signaling pathway Subtypes: VEGF-activated neuropilin signaling pathway involved in axon guidance [GO:1902378] Definition: The series of molecular signals initiated by vascular endothelial growth factor (VEGF) binding to a neuropilin protein on the surface of a target cell, and ending with the regulation of a downstream cellular process, e.g. transcription. References: PMID:12852851 Sources: GOC:BHF, GOC:rl Relationships: is a type of vascular endothelial growth factor signaling pathway [GO:0038084]; is a type of neuropilin signaling pathway [GO:0038189]; has part GO:0005021